positive regulation of hepatocyte apoptotic process [GO:1903945] (biological process) Relationships: is a type of regulation of hepatocyte apoptotic process [GO:1903943]; is a type of positive regulation of epithelial cell apoptotic process [GO:1904037]; RO_0002213 GO:0097284 Also known as: up regulation of hepatocyte apoptotic process, up-regulation of hepatocyte apoptotic process, upregulation of hepatocyte apoptotic process, activation of hepatocyte apoptosis, activation of hepatocyte apoptotic process, positive regulation of hepatocyte apoptosis, up regulation of hepatocyte apoptosis, up-regulation of hepatocyte apoptosis, upregulation of hepatocyte apoptosis References: PMID:8649852 Sources: GOC:TermGenie, GO_REF:0000058 Definition: Any process that activates or increases the frequency, rate or extent of hepatocyte apoptotic process.